{
  "term_label": "Unknown cellular component",
  "gene_symbol": "ASB3",
  "term_id": "UNKNOWN:0003",
  "gene_name": "Ankyrin repeat and SOCS box protein 3",
  "gene": "UniProtKB:Q9Y575"
}